{
  "gene_name": "Tissue factor pathway inhibitor 2",
  "term_label": "extracellular space",
  "gene": "UniProtKB:P48307",
  "gene_symbol": "TFPI2",
  "term_id": "GO:0005615"
}